{
  "gene": "UniProtKB:Q96RD6",
  "gene_name": "Pannexin-2",
  "term_id": "GO:0005886",
  "term_label": "plasma membrane",
  "gene_symbol": "PANX2"
}